{
  "term_label": "Unknown molecular function",
  "gene": "UniProtKB:Q96ES7",
  "gene_name": "SAGA-associated factor 29",
  "term_id": "UNKNOWN:0001",
  "gene_symbol": "SGF29"
}